{
  "gene_name": "V-type proton ATPase subunit B, brain isoform",
  "gene": "UniProtKB:P21281",
  "term_label": "vacuolar proton-transporting V-type ATPase, V1 domain",
  "gene_symbol": "ATP6V1B2",
  "term_id": "GO:0000221"
}